{
  "gene_symbol": "EBLN2",
  "term_id": "UNKNOWN:0001",
  "gene": "UniProtKB:Q6P2I7",
  "term_label": "Unknown molecular function",
  "gene_name": "Endogenous Bornavirus-like nucleoprotein 2"
}